{
  "gene": "UniProtKB:Q13950",
  "gene_symbol": "RUNX2",
  "gene_name": "Runt-related transcription factor 2",
  "term_label": "RNA polymerase II cis-regulatory region sequence-specific DNA binding",
  "term_id": "GO:0000978"
}